system development [GO:0048731] (biological process) Subtypes: skeletal system development [GO:0001501], urogenital system development [GO:0001655], GO:0001944, GO:0002520, nervous system development [GO:0007399], central nervous system development [GO:0007417], stomatogastric nervous system development [GO:0007421], peripheral nervous system development [GO:0007422], ventricular system development [GO:0021591], GO:0021761, preganglionic parasympathetic fiber development [GO:0021783], root system development [GO:0022622], endocrine system development [GO:0035270], exocrine system development [GO:0035272], GO:0048367, GO:0048483, enteric nervous system development [GO:0048484], sympathetic nervous system development [GO:0048485], parasympathetic nervous system development [GO:0048486], sensory system development [GO:0048880], digestive system development [GO:0055123], GO:0060037, GO:0060541, GO:0061008, reproductive system development [GO:0061458], GO:0072001, GO:0072359 Relationships: is a type of anatomical structure development [GO:0048856]; is part of multicellular organism development [GO:0007275] Sources: GOC:dph, GOC:jid Definition: The process whose specific outcome is the progression of an organismal system over time, from its formation to the mature structure. A system is a regularly interacting or interdependent group of organs or tissues that work together to carry out a given biological process.